{
  "gene_symbol": "ENTPD5",
  "gene_name": "Nucleoside diphosphate phosphatase ENTPD5",
  "term_id": "UNKNOWN:0003",
  "gene": "UniProtKB:O75356",
  "term_label": "Unknown cellular component"
}